2-methoxy-6-polyprenyl-1,4-benzoquinol methyltransferase activity [GO:0008425] (molecular function) References: PMID:23190198, PMID:9083048 Sources: RHEA:28286 Also known as: ubiquinone biosynthesis methyltransferase activity, ubiquinone biosynthetic process methyltransferase activity, 2-polyprenyl-6-methoxy-1,4-benzoquinone methylase activity, 2-polyprenyl-6-methoxy-1,4-benzoquinone methyltransferase activity, coenzyme Q biosynthesis methyltransferase activity, coenzyme Q biosynthetic process methyltransferase activity Definition: Catalysis of the reaction: a 2-methoxy-6-all-trans-polyprenyl-1,4-benzoquinol + S-adenosyl-L-methionine = a 6-methoxy-3-methyl-2-all-trans-polyprenyl-1,4-benzoquinol + S-adenosyl-L-homocysteine + H+. Relationships: is a type of GO:0008169; is part of GO:0006744 Note: Note that the polyprenyl sidechain substrate for this reaction has a different number of prenyl units in different organisms (for example, ubiquinone-6 in Saccharomyces, ubiquinone- 9 in rat and ubiquinone-10 in human), and thus the natural substrate for the enzymes from different organisms has a different number of prenyl units. However, the enzyme usually shows a low degree of specificity regarding the number of prenyl units.